{
  "term_label": "phosphomevalonate kinase activity",
  "gene_symbol": "PMVK",
  "gene_name": "Phosphomevalonate kinase",
  "gene": "UniProtKB:Q15126",
  "term_id": "GO:0004631"
}